{
  "term_label": "RNA polymerase II cis-regulatory region sequence-specific DNA binding",
  "term_id": "GO:0000978",
  "gene_symbol": "TAL2",
  "gene_name": "T-cell acute lymphocytic leukemia protein 2",
  "gene": "UniProtKB:Q16559"
}